fumagillin catabolic process [GO:1902085] (biological process) Also known as: fumagillin breakdown, fumagillin catabolism, fumagillin degradation Definition: The chemical reactions and pathways resulting in the breakdown of fumagillin. References: PMID:23488861 Sources: GOC:TermGenie, GOC:di Relationships: is a type of monocarboxylic acid catabolic process [GO:0072329]; is a type of epoxide metabolic process [GO:0097176]; is a type of ether catabolic process [GO:1901502]